negative regulation of fumonisin biosynthetic process [GO:1900684] (biological process) Definition: Any process that stops, prevents or reduces the frequency, rate or extent of fumonisin biosynthetic process. Sources: GOC:TermGenie, GOC:di Also known as: down regulation of fumonisin anabolism, down regulation of fumonisin biosynthesis, down regulation of fumonisin biosynthetic process, down regulation of fumonisin formation, down regulation of fumonisin synthesis, down-regulation of fumonisin anabolism, down-regulation of fumonisin biosynthesis, down-regulation of fumonisin biosynthetic process, down-regulation of fumonisin formation, down-regulation of fumonisin synthesis, downregulation of fumonisin anabolism, downregulation of fumonisin biosynthesis, downregulation of fumonisin biosynthetic process, downregulation of fumonisin formation, downregulation of fumonisin synthesis, inhibition of fumonisin anabolism, inhibition of fumonisin biosynthesis, inhibition of fumonisin formation, inhibition of fumonisin synthesis, negative regulation of fumonisin anabolism, negative regulation of fumonisin biosynthesis, negative regulation of fumonisin formation, negative regulation of fumonisin synthesis, inhibition of fumonisin biosynthetic process Relationships: is a type of negative regulation of small molecule metabolic process [GO:0062014]; is a type of GO:1900377; is_a regulation of fumonisin biosynthetic process [GO:1900683]; negatively regulates fumonisin biosynthetic process [GO:1900541]